{
  "term_id": "GO:0003729",
  "term_label": "mRNA binding",
  "gene": "UniProtKB:Q8NDT2",
  "gene_name": "Putative RNA-binding protein 15B",
  "gene_symbol": "RBM15B"
}